{
  "term_label": "centriole",
  "gene_symbol": "C2CD3",
  "gene_name": "C2 domain-containing protein 3",
  "term_id": "GO:0005814",
  "gene": "UniProtKB:Q4AC94"
}